{
  "term_label": "transforming growth factor beta receptor activity",
  "term_id": "GO:0005024",
  "gene_name": "Transforming growth factor-beta receptor type 3-like protein",
  "gene": "UniProtKB:H3BV60",
  "gene_symbol": "TGFBR3L"
}